tRNA (adenine(57)-N1)/(adenine(58)-N1)-methyltransferase activity [GO:0043827] (molecular function) Definition: Catalysis of the reaction: adenosine57/adenosine58 in tRNA + 2 S-adenosyl-L-methionine = 2 H+ + N1-methyladenosine57/N1-methyladenosine58 in tRNA + 2 S-adenosyl-L-homocysteine. References: PMID:14739239, PMID:20483913 Sources: RHEA:41740 Also known as: tRNA (adenine(57)-N(1))/(adenine(58)-N(1))-methyltransferase activity, tRNA (adenine(57)-N1-)/(adenine(58)-N1-)-methyltransferase activity, tRNA (adenine(57)-N1-/adenine(58)-N1-)-methyltransferase activity, tRNA (adenine-57, 58 N1-) methyltransferase activity, tRNA (adenine-57, 58-N(1)-) methyltransferase activity, tRNA (adenine-57, 58-N1-) methyltransferase activity Relationships: is a type of GO:0016426